{
  "gene_symbol": "DOCK1",
  "term_id": "GO:0005886",
  "gene_name": "Dedicator of cytokinesis protein 1",
  "term_label": "plasma membrane",
  "gene": "UniProtKB:Q14185"
}